{
  "term_id": "GO:0031514",
  "gene_name": "Centriole and centriolar satellite protein OFD1",
  "gene_symbol": "OFD1",
  "gene": "UniProtKB:O75665",
  "term_label": "motile cilium"
}